{
  "gene_name": "Cyclin-dependent kinase 5",
  "term_label": "synaptic vesicle transport",
  "gene_symbol": "CDK5",
  "gene": "UniProtKB:Q00535",
  "term_id": "GO:0048489"
}